cytosine transport [GO:0015856] (biological process) Relationships: is a type of pyrimidine nucleobase transport [GO:0015855] Sources: GOC:go_curators Definition: The directed movement of cytosine, 4-amino-2-hydroxypyrimidine, into, out of or within a cell, or between cells, by means of some agent such as a transporter or pore. Also known as: cytosine transmembrane transport